3-demethylubiquinone 3-O-methyltransferase activity [GO:0120537] (molecular function) Definition: Catalysis of the reaction: a 3-demethylubiquinone + S-adenosyl-L-methionine = a ubiquinone + S-adenosyl-L-homocysteine. References: PMID:38425362 Sources: RHEA:81215 Relationships: is a type of O-methyltransferase activity [GO:0008171]; is a type of S-adenosylmethionine-dependent methyltransferase activity [GO:0008757]; BFO_0000050 ubiquinone biosynthetic process [GO:0006744]